hydroxymethylfurfural reductase activity [GO:0033790] (molecular function) Definition: Catalysis of the reaction: 5-hydroxymethylfurfural + NAD(P)H + H+ = 2,5-bis-hydroxymethylfuran + NAD(P)+. References: PMID:15338422, PMID:16652391 Sources: GOC:jp, GOC:mah Relationships: is a type of oxidoreductase activity, acting on the CH-OH group of donors, NAD or NADP as acceptor [GO:0016616]